{
  "gene_symbol": "GRM5",
  "term_label": "plasma membrane",
  "term_id": "GO:0005886",
  "gene_name": "Metabotropic glutamate receptor 5",
  "gene": "UniProtKB:P41594"
}